{
  "gene_symbol": "RAG1",
  "term_label": "endodeoxyribonuclease complex",
  "gene": "UniProtKB:P15918",
  "term_id": "GO:1905347",
  "gene_name": "V(D)J recombination-activating protein 1"
}